ciliary basal body organization [GO:0032053] (biological process) Relationships: is a type of microtubule organizing center organization [GO:0031023]; is a type of cilium organization [GO:0044782] Definition: A process that is carried out at the cellular level which results in the assembly, arrangement of constituent parts, or disassembly of a ciliary basal body, a short cylindrical array of microtubules and associated proteins found at the base of a eukaryotic cilium (also called flagellum). Also known as: microtubule basal body organisation, microtubule basal body organization, microtubule basal body organization and biogenesis Subtypes: ciliary pro-basal body maturation [GO:0120311] References: PMID:9889124 Sources: GOC:cilia, GOC:dph, GOC:jl, GOC:krc, GOC:mah